{
  "term_id": "GO:0006457",
  "gene_name": "Peptidyl-prolyl cis-trans isomerase B",
  "gene_symbol": "PPIB",
  "gene": "UniProtKB:P23284",
  "term_label": "protein folding"
}